{
  "gene": "UniProtKB:Q5T6X4",
  "term_label": "Unknown molecular function",
  "gene_symbol": "FAM162B",
  "gene_name": "Protein FAM162B",
  "term_id": "UNKNOWN:0001"
}